axon extension involved in regeneration [GO:0048677] (BP) Definition: Long distance growth of a single axon process involved in regeneration of the neuron. Sources: GOC:jid Relationships: is a type of axon extension [GO:0048675]; is a type of sprouting of injured axon [GO:0048682] Regulation: regulated by regulation of axon extension involved in regeneration [GO:0048690]; RO_0002213 by GO:0048691; negatively regulated by negative regulation of axon extension involved in regeneration [GO:0048692]